hydrogen-sulfide S-acetyltransferase activity [GO:0047986] (molecular function) Relationships: is a type of S-acetyltransferase activity [GO:0016418] Also known as: hydrogen-sulphide S-acetyltransferase activity, acetyl-CoA:hydrogen-sulfide S-acetyltransferase activity, hydrogen-sulfide acetyltransferase activity Sources: EC:2.3.1.10, RHEA:16625 Definition: Catalysis of the reaction: acetyl-CoA + S(2-) = CoA + thioacetate.